regulation of chemokine production [GO:0032642] (biological process) Subtypes: regulation of fractalkine production [GO:0032644], negative regulation of chemokine production [GO:0032682], positive regulation of chemokine production [GO:0032722], regulation of chemokine (C-X-C motif) ligand 9 production [GO:0035394], regulation of chemokine (C-C motif) ligand 6 production [GO:0035531], regulation of monocyte chemotactic protein-1 production [GO:0071637], regulation of macrophage inflammatory protein 1 alpha production [GO:0071640], regulation of chemokine (C-C motif) ligand 4 production [GO:0071643], regulation of macrophage inflammatory protein-1 gamma production [GO:0071646], regulation of chemokine (C-C motif) ligand 5 production [GO:0071649], regulation of chemokine (C-C motif) ligand 1 production [GO:0071652], GO:0071658, regulation of chemokine (C-C motif) ligand 20 production [GO:1903884], GO:2000338, regulation of chemokine (C-X-C motif) ligand 2 production [GO:2000341] Definition: Any process that modulates the frequency, rate, or extent of chemokine production. Relationships: is a type of GO:0001817; RO_0002211 chemokine production [GO:0032602] Also known as: regulation of chemokine biosynthetic process, regulation of chemokine secretion Sources: GOC:mah